{
  "gene_symbol": "NAA25",
  "term_label": "acetyltransferase activator activity",
  "gene_name": "N-alpha-acetyltransferase 25, NatB auxiliary subunit",
  "gene": "UniProtKB:Q14CX7",
  "term_id": "GO:0010698"
}